{
  "gene_symbol": "TBC1D26",
  "gene": "UniProtKB:Q86UD7",
  "term_id": "UNKNOWN:0002",
  "gene_name": "TBC1 domain family member 26",
  "term_label": "Unknown biological process"
}